{
  "term_label": "Unknown biological process",
  "term_id": "UNKNOWN:0002",
  "gene_name": "Spermatogenesis associated 6-like protein",
  "gene_symbol": "SPATA6L",
  "gene": "UniProtKB:Q8N4H0"
}